{
  "term_id": "GO:0043001",
  "term_label": "Golgi to plasma membrane protein transport",
  "gene_name": "Phagosome assembly factor 1",
  "gene_symbol": "PHAF1",
  "gene": "UniProtKB:Q9BSU1"
}